{
  "gene_name": "Keratin-associated protein 12-4",
  "gene_symbol": "KRTAP12-4",
  "gene": "UniProtKB:P60329",
  "term_label": "Unknown biological process",
  "term_id": "UNKNOWN:0002"
}